coenzyme A transport [GO:0015880] (biological process) Relationships: is a type of organic anion transport [GO:0015711]; is a type of organophosphate ester transport [GO:0015748]; is a type of nucleobase-containing compound transport [GO:0015931]; is a type of amide transport [GO:0042886]; is a type of GO:0072348 Subtypes: coenzyme A transmembrane transport [GO:0035349] Definition: The directed movement of coenzyme A into, out of or within a cell, or between cells, by means of some agent such as a transporter or pore. Coenzyme A, 3'-phosphoadenosine-(5')diphospho(4')pantatheine, is an acyl carrier in many acylation and acyl-transfer reactions in which the intermediate is a thiol ester. Sources: GOC:ai